{
  "term_id": "UNKNOWN:0001",
  "term_label": "Unknown molecular function",
  "gene_symbol": "SPRR4",
  "gene_name": "Small proline-rich protein 4",
  "gene": "UniProtKB:Q96PI1"
}